{
  "term_label": "macrophage activation involved in immune response",
  "gene_symbol": "SYK",
  "gene": "UniProtKB:P43405",
  "gene_name": "Tyrosine-protein kinase SYK",
  "term_id": "GO:0002281"
}